{
  "gene_name": "Cleavage and polyadenylation specificity factor subunit 2",
  "gene_symbol": "CPSF2",
  "gene": "UniProtKB:Q9P2I0",
  "term_id": "GO:0003723",
  "term_label": "RNA binding"
}